{
  "gene_name": "Voltage-dependent calcium channel gamma-4 subunit",
  "gene": "UniProtKB:Q9UBN1",
  "term_label": "AMPA glutamate receptor complex",
  "term_id": "GO:0032281",
  "gene_symbol": "CACNG4"
}